nucleolar large rRNA transcription by RNA polymerase I [GO:0042790] (biological process) Relationships: is a type of transcription by RNA polymerase I [GO:0006360]; is a type of rRNA transcription [GO:0009303] Also known as: transcription of nuclear large rRNA transcript from RNA polymerase I promoter, transcription of nuclear rRNA large Pol I transcript, transcription of nucleolar large rRNA by RNA polymerase I Sources: GOC:jl, GOC:txnOH, ISBN:0321000382 Regulation: regulated by regulation of transcription of nucleolar large rRNA by RNA polymerase I [GO:1901836]; negatively regulated by negative regulation of transcription of nucleolar large rRNA by RNA polymerase I [GO:1901837]; positively regulated by positive regulation of transcription of nucleolar large rRNA by RNA polymerase I [GO:1901838] Definition: The synthesis of the large ribosomal RNA (rRNA) transcript which encodes several rRNAs, e.g. in mammals 28S, 18S and 5.8S, from a nuclear DNA template transcribed by RNA polymerase I.